negative regulation of protein modification process [GO:0031400] (biological process) Subtypes: negative regulation of protein phosphorylation [GO:0001933], negative regulation of protein glutathionylation [GO:0010734], negative regulation of peptidyl-lysine crotonylation [GO:0120094], GO:1900723, negative regulation of post-translational protein modification [GO:1901874], negative regulation of protein acetylation [GO:1901984], negative regulation of peptidyl-cysteine S-nitrosylation [GO:1902083], negative regulation of protein lipidation [GO:1903060], negative regulation of protein polyglycylation [GO:1903345], negative regulation of protein-pyridoxal-5-phosphate linkage [GO:1904286], negative regulation of tubulin deacetylation [GO:1904428], GO:1904807, negative regulation of protein geranylgeranylation [GO:2000540] Definition: Any process that stops, prevents, or reduces the frequency, rate or extent of the covalent alteration of one or more amino acid residues within a protein. Also known as: down regulation of protein modification, down-regulation of protein modification, downregulation of protein modification, inhibition of protein modification Relationships: is a type of regulation of protein modification process [GO:0031399]; is a type of GO:0051248; negatively regulates protein modification process [GO:0036211] Sources: GOC:mah, GOC:tb